{
  "term_label": "molybdopterin molybdotransferase activity",
  "gene": "UniProtKB:Q9NQX3",
  "gene_name": "Gephyrin",
  "term_id": "GO:0061599",
  "gene_symbol": "GPHN"
}